{
  "gene": "UniProtKB:Q16394",
  "term_id": "UNKNOWN:0002",
  "term_label": "Unknown biological process",
  "gene_symbol": "EXT1",
  "gene_name": "Exostosin-1"
}